{
  "term_label": "Unknown cellular component",
  "gene": "UniProtKB:A8K2U0",
  "term_id": "UNKNOWN:0003",
  "gene_symbol": "A2ML1",
  "gene_name": "Alpha-2-macroglobulin-like protein 1"
}